{
  "gene": "UniProtKB:Q96DU9",
  "gene_name": "Polyadenylate-binding protein 5",
  "term_label": "poly(U) RNA binding",
  "gene_symbol": "PABPC5",
  "term_id": "GO:0008266"
}